{
  "gene_name": "Oxysterols receptor LXR-alpha",
  "gene_symbol": "NR1H3",
  "gene": "UniProtKB:Q13133",
  "term_label": "RNA polymerase II cis-regulatory region sequence-specific DNA binding",
  "term_id": "GO:0000978"
}